negative regulation of trophectodermal cell proliferation [GO:1904074] (biological process) Definition: Any process that stops, prevents or reduces the frequency, rate or extent of trophectodermal cell proliferation. Also known as: down regulation of trophectoderm cell proliferation, down regulation of trophectodermal cell proliferation, down-regulation of trophectoderm cell proliferation, down-regulation of trophectodermal cell proliferation, downregulation of trophectoderm cell proliferation, downregulation of trophectodermal cell proliferation, negative regulation of trophectoderm cell proliferation, inhibition of trophectoderm cell proliferation, inhibition of trophectodermal cell proliferation References: PMID:24508636 Sources: GOC:TermGenie, GO_REF:0000058 Relationships: is a type of negative regulation of cell population proliferation [GO:0008285]; is a type of regulation of trophectodermal cell proliferation [GO:1904073]; negatively regulates trophectodermal cell proliferation [GO:0001834]